21U-RNA catabolic process [GO:0034586] (biological process) Also known as: 21U-RNA breakdown, 21U-RNA catabolism, 21U-RNA degradation Definition: The chemical reactions and pathways resulting in the breakdown of 21U-RNAs, a class of single-stranded RNA molecules of about 21 nucleotides in length characterized by a uridine 5'-monophosphate and a modified 3' end resistant to periodate degradation. 21U-RNAs are derived from distinct, autonomously expressed loci within the genome. Relationships: is a type of RNA catabolic process [GO:0006401]; is a type of 21U-RNA metabolic process [GO:0034585] Sources: GOC:kmv